{
  "gene_name": "Protein unc-13 homolog A",
  "term_id": "GO:0043195",
  "gene": "UniProtKB:Q9UPW8",
  "term_label": "terminal bouton",
  "gene_symbol": "UNC13A"
}